{
  "gene_symbol": "ADGRV1",
  "gene": "UniProtKB:Q8WXG9",
  "term_id": "GO:0004930",
  "gene_name": "Adhesion G-protein coupled receptor V1",
  "term_label": "G protein-coupled receptor activity"
}